ribitol catabolic process [GO:0046363] (BP) Definition: The chemical reactions and pathways resulting in the breakdown of ribitol, a pentitol derived formally by reduction of the -CHO group of either D- or L-ribose. Sources: ISBN:0198506732 Relationships: is_a pentitol catabolic process [GO:0019527] Subtypes: GO:0019488 Also known as: ribitol breakdown, ribitol catabolism, ribitol degradation